negative regulation of nitric oxide biosynthetic process [GO:0045019] (BP) Also known as: down regulation of nitric oxide biosynthetic process, down-regulation of nitric oxide biosynthetic process, downregulation of nitric oxide biosynthetic process, negative regulation of nitric oxide anabolism, negative regulation of nitric oxide biosynthesis, negative regulation of nitric oxide formation, negative regulation of nitric oxide synthesis, inhibition of nitric oxide biosynthetic process Definition: Any process that stops, prevents, or reduces the frequency, rate or extent of the chemical reactions and pathways resulting in the formation of nitric oxide. Sources: GOC:go_curators Relationships: is a type of GO:0009890; is a type of regulation of nitric oxide biosynthetic process [GO:0045428]; negatively regulates nitric oxide biosynthetic process [GO:0006809]